benzoyl-CoA metabolic process [GO:1901787] (BP) Definition: The chemical reactions and pathways involving benzoyl-CoA. Sources: GOC:TermGenie, GOC:yaf Also known as: benzoyl-CoA metabolism Relationships: is a type of acyl-CoA metabolic process [GO:0006637] Subtypes: benzoyl-CoA catabolic process [GO:1901788], benzoyl-CoA biosynthetic process [GO:1901789]